{
  "term_id": "UNKNOWN:0001",
  "gene_symbol": "PLET1",
  "term_label": "Unknown molecular function",
  "gene": "UniProtKB:Q6UQ28",
  "gene_name": "Placenta-expressed transcript 1 protein"
}